{
  "term_id": "UNKNOWN:0001",
  "gene_symbol": "ATXN7L3B",
  "gene": "UniProtKB:Q96GX2",
  "term_label": "Unknown molecular function",
  "gene_name": "Ataxin-7-like protein 3B"
}